neuron fate determination [GO:0048664] (biological process) Definition: The process in which a cell becomes capable of differentiating autonomously into a neuron regardless of its environment; upon determination, the cell fate cannot be reversed. Relationships: is a type of GO:0001709; is part of neuron fate commitment [GO:0048663] Sources: GOC:dph Subtypes: GO:0042668, photoreceptor cell fate determination [GO:0043703], ventral spinal cord interneuron fate determination [GO:0060580]